{
  "gene": "UniProtKB:Q6NXE6",
  "gene_symbol": "ARMC6",
  "gene_name": "Armadillo repeat-containing protein 6",
  "term_label": "hematopoietic progenitor cell differentiation",
  "term_id": "GO:0002244"
}